isopenicillin-N N-acyltransferase activity [GO:0050640] (molecular function) Definition: Catalysis of the reaction: phenylacetyl-CoA + isopenicillin N + H2O = CoA + penicillin G + L-2-aminoadipate. Relationships: is a type of N-acyltransferase activity [GO:0016410] Sources: RHEA:20720 Also known as: isopenicillin-N acyltransferase activity, acyl-CoA:isopenicillin N N-acyltransferase activity, acyl-coenzyme A:6-aminopenicillanic-acid-acyltransferase activity, acyl-coenzyme A:isopenicillin N acyltransferase activity, isopenicillin N:acyl-CoA acyltransferase activity